{
  "gene_name": "Tropomodulin-2",
  "term_id": "GO:0030016",
  "gene": "UniProtKB:Q9NZR1",
  "term_label": "myofibril",
  "gene_symbol": "TMOD2"
}